{
  "gene": "UniProtKB:P20700",
  "term_label": "nuclear migration",
  "gene_name": "Lamin-B1",
  "gene_symbol": "LMNB1",
  "term_id": "GO:0007097"
}